hair follicle maturation [GO:0048820] (biological process) Regulation: negatively regulated by negative regulation of hair follicle maturation [GO:0048817]; positively regulated by positive regulation of hair follicle maturation [GO:0048818]; regulated by regulation of hair follicle maturation [GO:0048819] Relationships: is a type of GO:0022405; is a type of GO:0071695; is part of hair follicle development [GO:0001942] Sources: GOC:devbiol Definition: A developmental process, independent of morphogenetic (shape) change, that is required for a hair follicle to attain its fully functional state.